queuine transmembrane transporter activity [GO:0160283] (molecular function) Definition: Enables the transfer of queuine from one side of a membrane to the other according to the reaction: queuine(out) = queuine(in). References: PMID:40526720 Relationships: is_a transmembrane transporter activity [GO:0022857]; is part of queuine import across plasma membrane [GO:0160284]